{
  "gene": "UniProtKB:Q08493",
  "term_label": "3',5'-cyclic-GMP phosphodiesterase activity",
  "gene_name": "cAMP-specific 3',5'-cyclic phosphodiesterase 4C",
  "term_id": "GO:0047555",
  "gene_symbol": "PDE4C"
}